{
  "term_label": "very long-chain fatty acid metabolic process",
  "term_id": "GO:0000038",
  "gene_name": "Long-chain-fatty-acid--CoA ligase 1",
  "gene_symbol": "ACSL1",
  "gene": "UniProtKB:P33121"
}